{
  "term_label": "positive regulation of mitochondrial membrane potential",
  "gene": "UniProtKB:Q8NCU8",
  "gene_name": "Mitoregulin",
  "term_id": "GO:0010918",
  "gene_symbol": "MTLN"
}